{
  "gene": "UniProtKB:P18075",
  "term_label": "cytokine activity",
  "gene_name": "Bone morphogenetic protein 7",
  "term_id": "GO:0005125",
  "gene_symbol": "BMP7"
}